D-glucose binding [GO:0005536] (molecular function) Relationships: is_a monosaccharide binding [GO:0048029] Sources: GOC:jl Definition: Binding to D-enantiomers of glucose. Also known as: glucose binding